response to mitotic DNA integrity checkpoint signaling [GO:1990820] (BP) Definition: A process that occurs in response to signals generated as a result of mitotic DNA integrity checkpoint signaling. References: PMID:7548844 Also known as: response to signal involved in mitotic DNA integrity checkpoint Relationships: is_a response to DNA integrity checkpoint signaling [GO:0072402]; is a type of GO:0072414